host cell wall [GO:0044158] (cellular component) Sources: GOC:rph Definition: The rigid or semi-rigid envelope lying outside the host cell membrane of plant, fungal, and most prokaryotic cells, maintaining their shape and protecting them from osmotic lysis. In plants it is made of cellulose and, often, lignin; in fungi it is composed largely of polysaccharides; in bacteria it is composed of peptidoglycan. Relationships: is a type of host cell part [GO:0033643]